{
  "gene_symbol": "RHOB",
  "term_id": "GO:0003924",
  "term_label": "GTPase activity",
  "gene": "UniProtKB:P62745",
  "gene_name": "Rho-related GTP-binding protein RhoB"
}